{
  "term_label": "MAP kinase tyrosine phosphatase activity",
  "gene_name": "Dual specificity protein phosphatase 9",
  "gene": "UniProtKB:Q99956",
  "term_id": "GO:0033550",
  "gene_symbol": "DUSP9"
}